regulation of intestinal epithelial cell development [GO:1905298] (biological process) Definition: Any process that modulates the frequency, rate or extent of intestinal epithelial cell development. References: PMID:23904268 Sources: GOC:BHF, GOC:BHF_miRNA, GOC:TermGenie, GOC:rph, GO_REF:0000058 Relationships: is a type of regulation of epithelial cell differentiation [GO:0030856]; is a type of regulation of cell development [GO:0060284]; regulates GO:0060576 Subtypes: GO:1905299, positive regulation of intestinal epithelial cell development [GO:1905300]